positive regulation of glial cell differentiation [GO:0045687] (biological process) Definition: Any process that activates or increases the frequency, rate or extent of glia cell differentiation. Relationships: is a type of positive regulation of gliogenesis [GO:0014015]; is a type of GO:0045685; positively regulates GO:0010001 Also known as: positive regulation of glia cell differentiation, positive regulation of neuroglia differentiation, up regulation of glial cell differentiation, up-regulation of glial cell differentiation, upregulation of glial cell differentiation, activation of glial cell differentiation, stimulation of glial cell differentiation Subtypes: positive regulation of microglia differentiation [GO:0014008], positive regulation of Schwann cell differentiation [GO:0014040], positive regulation of astrocyte differentiation [GO:0048711], positive regulation of oligodendrocyte differentiation [GO:0048714] Sources: GOC:go_curators